{
  "term_label": "Unknown biological process",
  "gene_symbol": "PCCA",
  "gene_name": "Propionyl-CoA carboxylase alpha chain, mitochondrial",
  "gene": "UniProtKB:P05165",
  "term_id": "UNKNOWN:0002"
}